{
  "term_id": "GO:0005764",
  "gene_symbol": "SMPD1",
  "gene": "UniProtKB:P17405",
  "gene_name": "Sphingomyelin phosphodiesterase",
  "term_label": "lysosome"
}